positive regulation of cGAS/STING signaling pathway [GO:0141111] (biological process) Relationships: is a type of GO:0039531; is_a GO:0062208; is a type of positive regulation of intracellular signal transduction [GO:1902533]; positively regulates cGAS/STING signaling pathway [GO:0140896] Definition: Any process that activates or increases the frequency, rate or extent of of cGAS/STING signaling pathway. References: PMID:37802025